{
  "term_id": "GO:0000785",
  "term_label": "chromatin",
  "gene": "UniProtKB:O15119",
  "gene_symbol": "TBX3",
  "gene_name": "T-box transcription factor TBX3"
}